hypoglossal nerve formation [GO:0021620] (biological process) Definition: The process that gives rise to the hypoglossal nerve. This process pertains to the initial formation of a structure from unspecified parts. This motor nerve innervates all the intrinsic and all but one of the extrinsic muscles of the tongue. Sources: GOC:cls, GOC:dgh, GOC:dph, GOC:jid, GO_REF:0000021 Also known as: CN XII biosynthesis, CN XII formation Relationships: is a type of cranial nerve formation [GO:0021603]; is part of hypoglossal nerve morphogenesis [GO:0021618]